{
  "gene": "UniProtKB:Q96EV8",
  "gene_symbol": "DTNBP1",
  "term_label": "BLOC-1 complex",
  "gene_name": "Dysbindin",
  "term_id": "GO:0031083"
}